{
  "term_id": "GO:0005634",
  "gene_name": "Proteasome subunit beta type-3",
  "gene_symbol": "PSMB3",
  "term_label": "nucleus",
  "gene": "UniProtKB:P49720"
}